{
  "gene_name": "Retinol dehydrogenase 11",
  "term_label": "Unknown molecular function",
  "gene_symbol": "RDH11",
  "term_id": "UNKNOWN:0001",
  "gene": "UniProtKB:Q8TC12"
}